{
  "gene_symbol": "IFRD1",
  "gene_name": "Interferon-related developmental regulator 1",
  "term_id": "GO:0005634",
  "term_label": "nucleus",
  "gene": "UniProtKB:O00458"
}